{
  "gene_symbol": "CDH5",
  "gene_name": "Cadherin-5",
  "gene": "UniProtKB:P33151",
  "term_label": "cell-cell junction assembly",
  "term_id": "GO:0007043"
}